{
  "gene_name": "Cytosolic phospholipase A2 delta",
  "term_label": "calcium-dependent phospholipid binding",
  "gene_symbol": "PLA2G4D",
  "gene": "UniProtKB:Q86XP0",
  "term_id": "GO:0005544"
}